{
  "gene_symbol": "PDE11A",
  "term_label": "negative regulation of cAMP/PKA signal transduction",
  "gene": "UniProtKB:Q9HCR9",
  "gene_name": "Dual 3',5'-cyclic-AMP and -GMP phosphodiesterase 11A",
  "term_id": "GO:0141162"
}